{
  "gene": "UniProtKB:A0A087WV62",
  "gene_symbol": "TRBV16",
  "term_label": "plasma membrane",
  "gene_name": "T cell receptor beta variable 16",
  "term_id": "GO:0005886"
}